tyramine signaling pathway [GO:0071928] (biological process) Regulation: regulated by regulation of tyramine signaling pathway [GO:2000131]; negatively regulated by negative regulation of tyramine signaling pathway [GO:2000132]; positively regulated by positive regulation of tyramine signaling pathway [GO:2000133] Relationships: is a type of octopamine or tyramine signaling pathway [GO:0007211] References: PMID:15355245 Sources: GOC:mah Definition: The series of molecular signals generated as a consequence of tyramine binding to a cell surface receptor. Also known as: tyramine signalling pathway